{
  "term_id": "GO:0005634",
  "term_label": "nucleus",
  "gene_symbol": "HDGFL1",
  "gene": "UniProtKB:Q5TGJ6",
  "gene_name": "Hepatoma-derived growth factor-like protein 1"
}